{
  "gene_symbol": "PRR34",
  "term_label": "Unknown molecular function",
  "gene_name": "Proline-rich protein 34",
  "gene": "UniProtKB:Q9NV39",
  "term_id": "UNKNOWN:0001"
}